respiratory chain complex I [GO:0045271] (cellular component) Definition: Respiratory chain complex I is an enzyme of the respiratory chain. It consists of several polypeptide chains and is L-shaped, with a horizontal arm lying in the membrane and a vertical arm that projects into the matrix. The electrons of NADH enter the chain at this complex. Note: Note that this term represents a location and not a function; the activity possessed by this complex is mentioned in the definition for the purpose of describing and distinguishing the complex. The function possessed by this complex is represented by the molecular function term 'NADH dehydrogenase (ubiquinone) activity ; GO:0008137'. Also known as: NADH dehydrogenase (ubiquinone) complex, NADH dehydrogenase complex (ubiquinone), NADH-Q oxidoreductase complex, electron transport complex I Relationships: is a type of NADH dehydrogenase complex [GO:0030964]; is a type of GO:0098803; is a type of transmembrane transporter complex [GO:1902495] Sources: GOC:imk, GOC:jid, ISBN:0716749556